{
  "gene": "UniProtKB:O75386",
  "term_label": "cilium",
  "gene_name": "Tubby-related protein 3",
  "term_id": "GO:0005929",
  "gene_symbol": "TULP3"
}